{
  "term_label": "Unknown molecular function",
  "gene": "UniProtKB:Q4U2R8",
  "gene_symbol": "SLC22A6",
  "term_id": "UNKNOWN:0001",
  "gene_name": "Solute carrier family 22 member 6"
}